low-affinity IgG receptor activity [GO:0019772] (molecular function) Relationships: is a type of IgG receptor activity [GO:0019770] Sources: GOC:add, GOC:signaling, ISBN:0781735149 Also known as: low affinity IgG receptor activity, low affinity Fc receptor activity Definition: Combining with low affinity with an immunoglobulin of an IgG isotype via the Fc region, and transmitting the signal from one side of the membrane to the other to initiate a change in cell activity.